{
  "gene_name": "Syntaxin-3",
  "term_label": "intracellular protein transport",
  "gene": "UniProtKB:Q13277",
  "gene_symbol": "STX3",
  "term_id": "GO:0006886"
}